{
  "gene": "UniProtKB:Q8NGX1",
  "gene_name": "Olfactory receptor 2T34",
  "term_id": "GO:0005886",
  "gene_symbol": "OR2T34",
  "term_label": "plasma membrane"
}